{
  "gene_symbol": "CHRNA3",
  "term_id": "GO:0051899",
  "gene_name": "Neuronal acetylcholine receptor subunit alpha-3",
  "gene": "UniProtKB:P32297",
  "term_label": "membrane depolarization"
}